{
  "gene_symbol": "HLA-DRA",
  "term_label": "late endosome membrane",
  "gene": "UniProtKB:P01903",
  "term_id": "GO:0031902",
  "gene_name": "HLA class II histocompatibility antigen, DR alpha chain"
}